somatic sensory system development [GO:0160038] (biological process) Definition: The process whose specific outcome is the progression of a somatic sensory system over time from its formation to the mature structure. Somatic sensory system is the sensory system for the sense of touch and pain. Relationships: is a type of GO:0048880 References: PMID:25832476, PMID:31399790 Also known as: somatosensory system development